{
  "gene_symbol": "GLRB",
  "gene": "UniProtKB:P48167",
  "term_id": "UNKNOWN:0003",
  "term_label": "Unknown cellular component",
  "gene_name": "Glycine receptor subunit beta"
}